{
  "gene_name": "Keratin-associated protein 10-10",
  "gene_symbol": "KRTAP10-10",
  "term_id": "UNKNOWN:0001",
  "term_label": "Unknown molecular function",
  "gene": "UniProtKB:P60014"
}